{
  "term_id": "UNKNOWN:0001",
  "term_label": "Unknown molecular function",
  "gene_symbol": "AATF",
  "gene_name": "Protein AATF",
  "gene": "UniProtKB:Q9NY61"
}